{
  "gene_name": "Holliday junction recognition protein",
  "gene_symbol": "HJURP",
  "term_id": "GO:0000775",
  "term_label": "chromosome, centromeric region",
  "gene": "UniProtKB:Q8NCD3"
}